{
  "term_id": "GO:0000242",
  "gene_symbol": "CEP192",
  "term_label": "pericentriolar material",
  "gene": "UniProtKB:Q8TEP8",
  "gene_name": "Centrosomal protein of 192 kDa"
}